{
  "gene_name": "High affinity immunoglobulin epsilon receptor subunit gamma",
  "term_label": "regulation of platelet activation",
  "gene_symbol": "FCER1G",
  "gene": "UniProtKB:P30273",
  "term_id": "GO:0010543"
}